UGA codon-amino acid adaptor activity [GO:0033415] (molecular function) Also known as: TGA codon-amino acid adaptor activity Definition: A triplet codon-amino acid adaptor activity that recognizes a UGA codon. Relationships: is_a triplet codon-amino acid adaptor activity [GO:0030533] Note: Note that in the standard genetic code, TGA is a stop codon (opal) and is not normally read by a tRNA. Sources: GOC:mah